female meiosis sister chromatid cohesion [GO:0007066] (biological process) Definition: The joining of the sister chromatids of a replicated chromosome along the entire length of the chromosome that occurs during meiosis in a female. Relationships: is a type of meiotic sister chromatid cohesion [GO:0051177] Sources: GOC:ai